{
  "gene_symbol": "ZNF480",
  "term_id": "GO:0005634",
  "term_label": "nucleus",
  "gene_name": "Zinc finger protein 480",
  "gene": "UniProtKB:Q8WV37"
}